regulation of pseudopodium assembly [GO:0031272] (biological process) Sources: GOC:pg Also known as: regulation of pseudopodium formation Definition: Any process that modulates the frequency, rate or extent of the assembly of pseudopodia. Subtypes: negative regulation of pseudopodium assembly [GO:0031273], positive regulation of pseudopodium assembly [GO:0031274] Relationships: is a type of GO:0120032; regulates pseudopodium assembly [GO:0031269]